{
  "gene_symbol": "PRSS41",
  "term_label": "plasma membrane",
  "term_id": "GO:0005886",
  "gene": "UniProtKB:Q7RTY9",
  "gene_name": "Serine protease 41"
}